{
  "gene": "UniProtKB:Q9Y2Z4",
  "term_label": "tyrosine-tRNA ligase activity",
  "gene_name": "Tyrosine--tRNA ligase, mitochondrial",
  "gene_symbol": "YARS2",
  "term_id": "GO:0004831"
}